{
  "term_id": "GO:0005741",
  "gene_symbol": "BCL2L2",
  "gene_name": "Bcl-2-like protein 2",
  "gene": "UniProtKB:Q92843",
  "term_label": "mitochondrial outer membrane"
}